{
  "gene_symbol": "SMAD1",
  "term_label": "transforming growth factor beta receptor signaling pathway",
  "gene": "UniProtKB:Q15797",
  "gene_name": "Mothers against decapentaplegic homolog 1",
  "term_id": "GO:0007179"
}